{
  "term_id": "GO:0098830",
  "gene": "UniProtKB:O14617",
  "term_label": "presynaptic endosome",
  "gene_name": "AP-3 complex subunit delta-1",
  "gene_symbol": "AP3D1"
}